{
  "term_label": "positive regulation of ERK5 cascade",
  "gene_name": "ALK and LTK ligand 1",
  "gene": "UniProtKB:Q6UXT8",
  "gene_symbol": "ALKAL1",
  "term_id": "GO:0070378"
}